negative regulation of granulocyte differentiation [GO:0030853] (biological process) Relationships: is a type of negative regulation of myeloid leukocyte differentiation [GO:0002762]; is a type of regulation of granulocyte differentiation [GO:0030852]; negatively regulates GO:0030851 Sources: GOC:mah Definition: Any process that stops, prevents, or reduces the frequency, rate or extent of granulocyte differentiation. Also known as: down regulation of granulocyte differentiation, down-regulation of granulocyte differentiation, downregulation of granulocyte differentiation, inhibition of granulocyte differentiation Subtypes: negative regulation of basophil differentiation [GO:0045641], negative regulation of eosinophil differentiation [GO:0045644], negative regulation of neutrophil differentiation [GO:0045659]